{
  "term_id": "GO:0034501",
  "term_label": "protein localization to kinetochore",
  "gene": "UniProtKB:Q96DY7",
  "gene_symbol": "MTBP",
  "gene_name": "Mdm2-binding protein"
}